{
  "gene_symbol": "TUBA4B",
  "gene": "UniProtKB:Q9H853",
  "term_id": "UNKNOWN:0002",
  "term_label": "Unknown biological process",
  "gene_name": "Putative tubulin-like protein alpha-4B"
}